{
  "term_id": "GO:0003730",
  "gene": "UniProtKB:P11940",
  "gene_name": "Polyadenylate-binding protein 1",
  "term_label": "mRNA 3'-UTR binding",
  "gene_symbol": "PABPC1"
}